{
  "gene_symbol": "KRT17",
  "term_id": "GO:0045109",
  "term_label": "intermediate filament organization",
  "gene": "UniProtKB:Q04695",
  "gene_name": "Keratin, type I cytoskeletal 17"
}